{
  "gene_name": "Hairy_enhancer-of-split related with YRPW motif protein 1",
  "term_id": "GO:0009952",
  "term_label": "anterior/posterior pattern specification",
  "gene": "UniProtKB:Q9Y5J3",
  "gene_symbol": "HEY1"
}